{
  "gene_symbol": "GART",
  "gene_name": "Trifunctional purine biosynthetic protein adenosine-3",
  "term_id": "GO:0006164",
  "term_label": "purine nucleotide biosynthetic process",
  "gene": "UniProtKB:P22102"
}